{
  "term_label": "protein insertion into mitochondrial inner membrane from matrix",
  "gene": "UniProtKB:Q9Y276",
  "gene_symbol": "BCS1L",
  "term_id": "GO:0032979",
  "gene_name": "Mitochondrial chaperone BCS1"
}